{
  "gene_symbol": "NOTCH2",
  "term_id": "GO:0009986",
  "gene_name": "Neurogenic locus notch homolog protein 2",
  "gene": "UniProtKB:Q04721",
  "term_label": "cell surface"
}